{
  "term_id": "GO:0005737",
  "gene_name": "Methionine-R-sulfoxide reductase B3",
  "gene_symbol": "MSRB3",
  "term_label": "cytoplasm",
  "gene": "UniProtKB:Q8IXL7"
}